nematode larval development [GO:0002119] (biological process) Sources: GOC:ems, GOC:kmv Regulation: regulated by regulation of nematode larval development [GO:0061062]; positively regulated by positive regulation of nematode larval development [GO:0061063]; negatively regulated by negative regulation of nematode larval development [GO:0061064] Subtypes: dauer larval development [GO:0040024] Definition: The process whose specific outcome is the progression of the nematode larva over time, from its formation to the mature structure. Nematode larval development begins with the newly hatched first-stage larva (L1) and ends with the end of the last larval stage (for example the fourth larval stage (L4) in C. elegans). Each stage of nematode larval development is characterized by proliferation of specific cell lineages and an increase in body size without alteration of the basic body plan. Nematode larval stages are separated by molts in which each stage-specific exoskeleton, or cuticle, is shed and replaced anew. Relationships: is a type of GO:0002164